{
  "term_label": "mitochondrion",
  "gene_symbol": "SLC25A38",
  "gene_name": "Mitochondrial glycine transporter",
  "gene": "UniProtKB:Q96DW6",
  "term_id": "GO:0005739"
}